actin filament bundle of actin-based cell projection [GO:0098859] (cellular component) Definition: A bundle of cross-linked actin filaments that is part of an actin-based cell protrusion, in which filaments are oriented such that the plus (barbed) ends are at the tip of the protrusion, capped by a tip complex which stabilizes the filaments. References: PMID:12566431, PMID:15661519 Relationships: is a type of GO:0097518; is part of actin-based cell projection [GO:0098858] Subtypes: microvillar actin bundle [GO:0097516], GO:0098860, actin filament bundle of filopodium [GO:0098861]